{
  "gene_name": "Apelin receptor",
  "term_label": "blood vessel development",
  "gene": "UniProtKB:P35414",
  "gene_symbol": "APLNR",
  "term_id": "GO:0001568"
}